{
  "gene_name": "Dual specificity phosphatase 28",
  "term_label": "Unknown biological process",
  "gene_symbol": "DUSP28",
  "gene": "UniProtKB:Q4G0W2",
  "term_id": "UNKNOWN:0002"
}